arginyl-tRNA aminoacylation [GO:0006420] (biological process) Subtypes: GO:0070144 Relationships: is a type of tRNA aminoacylation for protein translation [GO:0006418] Sources: GOC:mcc, ISBN:0716730510 Definition: The process of coupling arginine to arginyl-tRNA, catalyzed by arginyl-tRNA synthetase. The arginyl-tRNA synthetase is a class-I synthetase. The activated amino acid is transferred to the 2'-OH group of an alanine accetping tRNA. The 2'-O-aminoacyl-tRNA will ultimately migrate to the 3' position via transesterification.